loop of Henle development [GO:0072070] (biological process) Sources: GOC:mtg_kidney_jan10 Also known as: intermediate tubule development Subtypes: metanephric loop of Henle development [GO:0072236] Definition: The process whose specific outcome is the progression of the loop of Henle over time, from its formation to the mature structure. The loop of Henle is a nephron tubule that connects the proximal convoluted tubule to the distal convoluted tubule. Relationships: is a type of GO:0072080